{
  "gene": "UniProtKB:Q5T4F4",
  "gene_name": "Protrudin",
  "term_label": "endoplasmic reticulum tubular network formation",
  "gene_symbol": "ZFYVE27",
  "term_id": "GO:0071787"
}